{
  "gene": "UniProtKB:A8MUP6",
  "gene_name": "Germ cell-specific gene 1-like protein 2",
  "term_label": "Unknown molecular function",
  "gene_symbol": "GSG1L2",
  "term_id": "UNKNOWN:0001"
}